3-hydroxyisobutyryl-CoA hydrolase activity [GO:0003860] (molecular function) Definition: Catalysis of the reaction: 3-hydroxy-2-methylpropanoyl-CoA + H2O = CoA + 3-hydroxy-2-methylpropanoate. Sources: EC:3.1.2.4 Also known as: 3-hydroxy-2-methylpropanoyl-CoA hydrolase activity, 3-hydroxy-isobutyryl CoA hydrolase activity, HIB CoA deacylase activity Relationships: is a type of short-chain fatty acyl-CoA hydrolase activity [GO:0141126]